{
  "gene": "UniProtKB:P04054",
  "term_id": "GO:0005543",
  "gene_name": "Phospholipase A2",
  "gene_symbol": "PLA2G1B",
  "term_label": "phospholipid binding"
}